{
  "gene_symbol": "ARL4A",
  "gene": "UniProtKB:P40617",
  "gene_name": "ADP-ribosylation factor-like protein 4A",
  "term_label": "plasma membrane",
  "term_id": "GO:0005886"
}